{
  "gene_name": "Dolichyl-diphosphooligosaccharide--protein glycosyltransferase subunit 1",
  "gene": "UniProtKB:P04843",
  "term_label": "oligosaccharyltransferase complex",
  "term_id": "GO:0008250",
  "gene_symbol": "RPN1"
}